{
  "term_label": "regulation of transcription by RNA polymerase II",
  "gene_symbol": "HOPX",
  "gene_name": "Homeodomain-only protein",
  "term_id": "GO:0006357",
  "gene": "UniProtKB:Q9BPY8"
}